{
  "gene": "UniProtKB:Q9Y2E4",
  "gene_name": "Disco-interacting protein 2 homolog C",
  "term_id": "UNKNOWN:0002",
  "term_label": "Unknown biological process",
  "gene_symbol": "DIP2C"
}